{
  "term_id": "GO:0008535",
  "gene_symbol": "COA7",
  "term_label": "respiratory chain complex IV assembly",
  "gene": "UniProtKB:Q96BR5",
  "gene_name": "Cytochrome c oxidase assembly factor 7"
}